{
  "gene_name": "Coiled-coil domain-containing protein 175",
  "term_label": "Unknown molecular function",
  "term_id": "UNKNOWN:0001",
  "gene_symbol": "CCDC175",
  "gene": "UniProtKB:P0C221"
}